{
  "gene": "UniProtKB:P16109",
  "term_label": "leukocyte tethering or rolling",
  "term_id": "GO:0050901",
  "gene_name": "P-selectin",
  "gene_symbol": "SELP"
}